{
  "gene_name": "Exocyst complex component 1",
  "term_label": "Golgi to plasma membrane transport",
  "gene_symbol": "EXOC1",
  "gene": "UniProtKB:Q9NV70",
  "term_id": "GO:0006893"
}